positive regulation of xylose catabolic process to ethanol [GO:1900517] (biological process) Sources: GOC:TermGenie, GOC:mengo_curators Definition: Any process that activates or increases the frequency, rate or extent of xylose catabolic process to ethanol. Relationships: is a type of positive regulation of catabolic process [GO:0009896]; is a type of GO:0045913; is a type of GO:0062013; is a type of GO:1900515; positively regulates D-xylose catabolic process to ethanol [GO:0044577] Also known as: activation of xylose catabolism to ethanol, positive regulation of xylose catabolism to ethanol, up regulation of xylose catabolic process to ethanol, up regulation of xylose catabolism to ethanol, up-regulation of xylose catabolic process to ethanol, up-regulation of xylose catabolism to ethanol, upregulation of xylose catabolic process to ethanol, upregulation of xylose catabolism to ethanol, activation of xylose catabolic process to ethanol